negative regulation of T-helper 17 type immune response [GO:2000317] (biological process) Relationships: is a type of negative regulation of adaptive immune response based on somatic recombination of immune receptors built from immunoglobulin superfamily domains [GO:0002823]; is a type of regulation of T-helper 17 type immune response [GO:2000316]; negatively regulates T-helper 17 type immune response [GO:0072538] Subtypes: negative regulation of T-helper 17 cell differentiation [GO:2000320] Definition: Any process that stops, prevents or reduces the frequency, rate or extent of T-helper 17 type immune response. Also known as: negative regulation of Th17 immune response Sources: GOC:BHF, GOC:mah